{
  "gene_symbol": "PLEKHA8",
  "gene": "UniProtKB:Q96JA3",
  "gene_name": "Pleckstrin homology domain-containing family A member 8",
  "term_id": "GO:0120009",
  "term_label": "intermembrane lipid transfer"
}